epidermal growth factor signaling pathway involved in forebrain neuron fate commitment [GO:0022026] (biological process) Sources: GOC:cls, GOC:dgh, GOC:dph, GOC:jid, GO_REF:0000021 Definition: The series of molecular signals generated as a consequence of a epidermal growth factor receptor binding to one of its physiological ligands that contributes to the commitment of a neuroblast to a neuronal fate. The neuron will reside in the forebrain. Relationships: is a type of epidermal growth factor receptor signaling pathway [GO:0007173]; is part of commitment of multipotent stem cells to neuronal lineage in forebrain [GO:0021898] Also known as: epidermal growth factor signalling pathway involved in forebrain neuron fate commitment